protein K29-linked deubiquitination [GO:0035523] (biological process) Relationships: is a type of protein deubiquitination [GO:0016579] Sources: GOC:bf Definition: A protein deubiquitination process in which a K29-linked ubiquitin chain, i.e. a polymer of ubiquitin formed by linkages between lysine residues at position 29 of the ubiquitin monomers, is removed from a protein. Also known as: protein K29-linked deubiquitinylation, protein K29-linked deubiquitylation